regulation of cell projection assembly [GO:0060491] (biological process) Subtypes: regulation of plasma membrane bounded cell projection assembly [GO:0120032], GO:1902208, regulation of type IV pilus biogenesis [GO:1903656] Also known as: regulation of cell projection formation Sources: GOC:dph, GOC:tb Relationships: is a type of GO:0031344; is a type of GO:0044087; regulates cell projection assembly [GO:0030031] Definition: Any process that modulates the rate, frequency, or extent of cell projection assembly.